{
  "term_id": "GO:0060070",
  "gene_symbol": "DIXDC1",
  "gene": "UniProtKB:Q155Q3",
  "gene_name": "Dixin",
  "term_label": "canonical Wnt signaling pathway"
}